{
  "gene_symbol": "SPOPL",
  "term_id": "GO:0005737",
  "term_label": "cytoplasm",
  "gene_name": "Speckle-type POZ protein-like",
  "gene": "UniProtKB:Q6IQ16"
}